{
  "term_label": "cytosol",
  "term_id": "GO:0005829",
  "gene_symbol": "HDAC10",
  "gene_name": "Polyamine deacetylase HDAC10",
  "gene": "UniProtKB:Q969S8"
}